{
  "term_label": "ribosomal subunit export from nucleus",
  "gene_name": "Eukaryotic translation initiation factor 6",
  "term_id": "GO:0000054",
  "gene_symbol": "EIF6",
  "gene": "UniProtKB:P56537"
}